response to pheromone [GO:0019236] (biological process) Sources: GOC:jl Subtypes: response to pheromone regulating pheromone-induced unidirectional conjugation [GO:0000765], detection of pheromone [GO:0043695], GO:0071444 Also known as: pheromone response Relationships: is a type of response to chemical [GO:0042221] Definition: Any process that results in a change in state or activity of a cell or an organism (in terms of movement, secretion, enzyme production, gene expression, etc.) as a result of a pheromone stimulus.